{
  "term_label": "dynein heavy chain binding",
  "term_id": "GO:0045504",
  "gene": "UniProtKB:O14645",
  "gene_name": "Axonemal dynein light intermediate polypeptide 1",
  "gene_symbol": "DNALI1"
}